regulation of arginine catabolic process [GO:1900081] (biological process) Also known as: regulation of arginine breakdown, regulation of arginine catabolism, regulation of arginine degradation Definition: Any process that modulates the frequency, rate or extent of arginine catabolic process. Subtypes: GO:1900082 Relationships: is a type of regulation of amino acid metabolic process [GO:0006521]; is a type of regulation of amine catabolic process [GO:0033241]; is a type of regulation of small molecule metabolic process [GO:0062012]; regulates L-arginine catabolic process [GO:0006527] Sources: GOC:TermGenie, GOC:dgf